negative regulation of epidermal growth factor-activated receptor activity [GO:0007175] (biological process) Definition: Any process that stops, prevents, or reduces the frequency, rate or extent of EGF-activated receptor activity. Sources: GOC:go_curators Relationships: is a type of GO:0042059; is a type of negative regulation of protein tyrosine kinase activity [GO:0061099]; is a type of negative regulation of signaling receptor activity [GO:2000272]; negatively regulates epidermal growth factor receptor activity [GO:0005006] Also known as: EGF receptor downregulation, down regulation of epidermal growth factor receptor activity, down-regulation of epidermal growth factor receptor activity, downregulation of epidermal growth factor receptor activity, negative regulation of EGF receptor activity, negative regulation of EGFR activity, negative regulation of epidermal growth factor receptor activity, inhibition of epidermal growth factor receptor activity